pronephric nephron development [GO:0039019] (biological process) Definition: The process whose specific outcome is the progression of the pronephric nephron over time, from its formation to the mature structure. A pronephric nephron is the functional unit of the pronephros. Sources: GOC:mtg_kidney_jan10, XAO:00002785 Relationships: is a type of GO:0072006; is part of pronephros development [GO:0048793]